{
  "gene": "UniProtKB:Q99567",
  "term_label": "Unknown molecular function",
  "gene_symbol": "NUP88",
  "gene_name": "Nuclear pore complex protein Nup88",
  "term_id": "UNKNOWN:0001"
}